specification of pronephric proximal tubule identity [GO:0039004] (biological process) Relationships: is a type of specification of pronephric tubule identity [GO:0039005]; is_a specification of proximal tubule identity [GO:0072082]; is a type of proximal/distal pattern formation involved in pronephric nephron development [GO:0072196]; is part of GO:0039011 Definition: The process in which the proximal tubule of the pronephric nephron acquires its identity. Sources: GOC:mtg_kidney_jan10